{
  "term_label": "centrosome",
  "gene_symbol": "CENPJ",
  "term_id": "GO:0005813",
  "gene_name": "Centromere protein J",
  "gene": "UniProtKB:Q9HC77"
}